protein localization to phagocytic vesicle [GO:1905161] (biological process) Relationships: is a type of protein localization to organelle [GO:0033365] Also known as: protein localisation in phagocytic vesicle, protein localisation to phagocytic vesicle, protein localisation to phagosome, protein localization in phagocytic vesicle, protein recruitment to phagosome Definition: A process in which a protein is transported to, or maintained in, a location within a phagocytic vesicle. References: PMID:23303671 Sources: GOC:PARL, GOC:TermGenie, GOC:bf, GO_REF:0000087 Regulation: regulated by regulation of protein localization to phagocytic vesicle [GO:1905169]; negatively regulated by negative regulation of protein localization to phagocytic vesicle [GO:1905170]; positively regulated by GO:1905171